{
  "gene": "UniProtKB:Q9NRN7",
  "term_id": "GO:0019878",
  "term_label": "lysine biosynthetic process via aminoadipic acid",
  "gene_name": "L-aminoadipate-semialdehyde dehydrogenase-phosphopantetheinyl transferase",
  "gene_symbol": "AASDHPPT"
}